{
  "term_id": "GO:0043495",
  "gene_symbol": "SUN5",
  "gene": "UniProtKB:Q8TC36",
  "gene_name": "SUN domain-containing protein 5",
  "term_label": "protein-membrane adaptor activity"
}